{
  "gene": "UniProtKB:O15264",
  "term_label": "protein serine/threonine kinase activity",
  "gene_symbol": "MAPK13",
  "gene_name": "Mitogen-activated protein kinase 13",
  "term_id": "GO:0004674"
}